{
  "gene": "UniProtKB:A8MVS5",
  "term_id": "UNKNOWN:0003",
  "term_label": "Unknown cellular component",
  "gene_symbol": "HIDE1",
  "gene_name": "Protein HIDE1"
}